{
  "gene": "UniProtKB:Q8N163",
  "term_id": "GO:0000774",
  "gene_name": "Cell cycle and apoptosis regulator protein 2",
  "gene_symbol": "CCAR2",
  "term_label": "adenyl-nucleotide exchange factor activity"
}